ascospore release from ascus [GO:0071998] (biological process) Relationships: is a type of developmental process involved in reproduction [GO:0003006]; is a type of GO:0048869; is a type of meiotic cell cycle process [GO:1903046]; is part of sexual sporulation resulting in formation of a cellular spore [GO:0043935] Definition: A developmental process that results in the discharge of ascospores from the ascus. Ascospore release may be active or passive. Also known as: ascospore liberation Sources: DOI:10.1016/S0953-7562(96)80057-8, GOC:mah